{
  "gene": "UniProtKB:Q8TBM7",
  "gene_name": "Transmembrane protein 254",
  "term_id": "UNKNOWN:0001",
  "gene_symbol": "TMEM254",
  "term_label": "Unknown molecular function"
}